host peribacteroid membrane [GO:0043664] (cellular component) Definition: A host-derived membrane that surrounds one or more bacteroids (such as nitrogen-fixing bacteroids within legume root nodule cells). Relationships: is a type of GO:0033643; is part of host bacteroid-containing symbiosome [GO:0043663] Sources: GOC:cc